{
  "gene_symbol": "SUMO1P1",
  "gene_name": "Small ubiquitin-related modifier 5",
  "term_id": "GO:0005634",
  "term_label": "nucleus",
  "gene": "UniProtKB:G2XKQ0"
}